{
  "gene_name": "Ferredoxin-2, mitochondrial",
  "term_id": "GO:0009055",
  "gene": "UniProtKB:Q6P4F2",
  "gene_symbol": "FDX2",
  "term_label": "electron transfer activity"
}